interneuron-substratum interaction involved in interneuron migration from the subpallium to the cortex [GO:0021839] (biological process) Definition: The process in which migrating interneurons interact with an external substratum as a component of migration from the subpallium to the cortex. References: PMID:12626695 Sources: GOC:cls, GOC:dgh, GOC:dph, GOC:jid, GO_REF:0000021 Relationships: is a type of cell-substrate adhesion [GO:0031589]; is part of GO:0021830